{
  "gene_name": "WASH complex subunit 4",
  "term_id": "GO:0016197",
  "term_label": "endosomal transport",
  "gene_symbol": "WASHC4",
  "gene": "UniProtKB:Q2M389"
}